{
  "gene": "UniProtKB:O75771",
  "gene_name": "DNA repair protein RAD51 homolog 4",
  "term_id": "GO:0007131",
  "gene_symbol": "RAD51D",
  "term_label": "reciprocal meiotic recombination"
}